{
  "gene": "UniProtKB:P04259",
  "term_id": "GO:0031424",
  "gene_name": "Keratin, type II cytoskeletal 6B",
  "gene_symbol": "KRT6B",
  "term_label": "keratinization"
}